{
  "term_label": "DNA-binding transcription factor activity, RNA polymerase II-specific",
  "term_id": "GO:0000981",
  "gene": "UniProtKB:P17041",
  "gene_name": "Zinc finger protein 32",
  "gene_symbol": "ZNF32"
}